response to prostaglandin I [GO:0034697] (biological process) Sources: GOC:BHF, GOC:vk Also known as: response to prostaglandin I stimulus Definition: Any process that results in a change in state or activity of a cell or an organism (in terms of movement, secretion, enzyme production, gene expression, etc.) as a result of a prostagladin I stimulus. Subtypes: GO:0071382 Relationships: is a type of response to prostaglandin [GO:0034694]; is a type of response to oxygen-containing compound [GO:1901700]